{
  "term_label": "cell adhesion molecule binding",
  "term_id": "GO:0050839",
  "gene_symbol": "PCDHGB1",
  "gene_name": "Protocadherin gamma-B1",
  "gene": "UniProtKB:Q9Y5G3"
}